synaptic transmission involved in micturition [GO:0060084] (biological process) Also known as: synaptic transmission involved in urination Relationships: is a type of neuromuscular synaptic transmission [GO:0007274]; is part of micturition [GO:0060073] Definition: The process of communication from a neuron to a smooth muscle in the bladder that contributes to the expulsion of urine from the body. References: PMID:15827347 Sources: GOC:dph